{
  "term_label": "cytoplasm",
  "gene": "UniProtKB:Q5SZQ8",
  "gene_name": "CUGBP Elav-like family member 3",
  "gene_symbol": "CELF3",
  "term_id": "GO:0005737"
}